{
  "gene_name": "Noggin",
  "gene_symbol": "NOG",
  "term_id": "GO:0009953",
  "term_label": "dorsal/ventral pattern formation",
  "gene": "UniProtKB:Q13253"
}